{
  "gene_name": "Putative homeobox protein NANOG2",
  "gene_symbol": "NANOGP1",
  "gene": "UniProtKB:Q8N7R0",
  "term_label": "cell differentiation",
  "term_id": "GO:0030154"
}